{
  "gene_symbol": "PDCD7",
  "gene": "UniProtKB:Q8N8D1",
  "term_label": "Unknown molecular function",
  "term_id": "UNKNOWN:0001",
  "gene_name": "Programmed cell death protein 7"
}